{
  "gene": "UniProtKB:Q9BWF2",
  "term_id": "GO:0090734",
  "gene_symbol": "TRAIP",
  "gene_name": "E3 ubiquitin-protein ligase TRAIP",
  "term_label": "site of DNA damage"
}